regulation of synergid differentiation [GO:0045697] (BP) Also known as: regulation of synergid cell differentiation Sources: GOC:go_curators Definition: Any process that modulates the frequency, rate or extent of synergid cell differentiation. Subtypes: negative regulation of synergid differentiation [GO:0045698], positive regulation of synergid differentiation [GO:0045699] Relationships: is a type of regulation of cell differentiation [GO:0045595]; regulates GO:0009563